{
  "term_id": "GO:0004713",
  "term_label": "protein tyrosine kinase activity",
  "gene_name": "Tyrosine-protein kinase SYK",
  "gene_symbol": "SYK",
  "gene": "UniProtKB:P43405"
}